{
  "term_label": "extracellular space",
  "gene_symbol": "ENG",
  "gene_name": "Endoglin",
  "gene": "UniProtKB:P17813",
  "term_id": "GO:0005615"
}